{
  "gene": "UniProtKB:Q07001",
  "gene_name": "Acetylcholine receptor subunit delta",
  "gene_symbol": "CHRND",
  "term_id": "GO:0051899",
  "term_label": "membrane depolarization"
}